{
  "gene_symbol": "BST2",
  "term_label": "innate immune response",
  "term_id": "GO:0045087",
  "gene_name": "Bone marrow stromal antigen 2",
  "gene": "UniProtKB:Q10589"
}